{
  "term_label": "microtubule associated complex",
  "gene": "UniProtKB:P46821",
  "term_id": "GO:0005875",
  "gene_name": "Microtubule-associated protein 1B",
  "gene_symbol": "MAP1B"
}